{
  "term_id": "GO:0045321",
  "gene_symbol": "PRDX2",
  "term_label": "leukocyte activation",
  "gene_name": "Peroxiredoxin-2",
  "gene": "UniProtKB:P32119"
}